purine deoxyribonucleoside monophosphate catabolic process [GO:0009172] (biological process) Relationships: is a type of purine nucleoside monophosphate catabolic process [GO:0009128]; is a type of deoxyribonucleoside monophosphate catabolic process [GO:0009159]; is a type of purine deoxyribonucleoside monophosphate metabolic process [GO:0009170] Definition: The chemical reactions and pathways resulting in the breakdown of purine deoxyribonucleoside monophosphate, a compound consisting of a purine base linked to a deoxyribose sugar esterified with phosphate on the sugar. Also known as: purine deoxyribonucleoside monophosphate breakdown, purine deoxyribonucleoside monophosphate catabolism, purine deoxyribonucleoside monophosphate degradation Subtypes: GO:0046055, dAMP catabolic process [GO:0046059] Sources: GOC:go_curators, ISBN:0198506732